protein transporter activity [GO:0140318] (molecular function) Subtypes: protein transmembrane transporter activity [GO:0008320], lipoprotein releasing activity [GO:0140306], GO:0140567 Also known as: protein carrier activity, protein transport chaperone Definition: Directly binding to a specific protein and delivering it to a specific cellular location. Relationships: is a type of transporter activity [GO:0005215] References: PMID:18706423 Note: Examples of protein carriers include the soluble TIM chaperone complexes of S. cerevisiae Tim9-Tim10 and Tim8-Tim13, that provide a shuttle system between TOM and the membrane insertases TIM22 and SAM and, thus, ensure that precursors are kept in a translocation-competent conformation.